{
  "term_id": "GO:0005829",
  "gene": "UniProtKB:P15559",
  "term_label": "cytosol",
  "gene_name": "NAD(P)H dehydrogenase [quinone] 1",
  "gene_symbol": "NQO1"
}